{
  "gene_symbol": "ATP5ME",
  "gene_name": "ATP synthase subunit e, mitochondrial",
  "term_label": "proton-transporting ATP synthase activity, rotational mechanism",
  "term_id": "GO:0046933",
  "gene": "UniProtKB:P56385"
}